glycolate catabolic process [GO:0046296] (biological process) Sources: GOC:ai Also known as: glycolate breakdown, glycolate catabolism, glycolate degradation Relationships: is_a glycolate metabolic process [GO:0009441]; is a type of primary alcohol catabolic process [GO:0034310]; is a type of monocarboxylic acid catabolic process [GO:0072329] Definition: The chemical reactions and pathways resulting in the breakdown of glycolate, the anion of hydroxyethanoic acid (glycolic acid).